{
  "term_label": "inositol hexakisphosphate kinase activity",
  "term_id": "GO:0000828",
  "gene_name": "Inositol hexakisphosphate and diphosphoinositol-pentakisphosphate kinase 2",
  "gene_symbol": "PPIP5K2",
  "gene": "UniProtKB:O43314"
}